periplasmic space [GO:0042597] (cellular component) Relationships: is a type of cellular anatomical structure [GO:0110165] Sources: GOC:go_curators, GOC:md Definition: The region between the inner (cytoplasmic) and outer membrane (Gram-negative Bacteria) or cytoplasmic membrane and cell wall (Fungi and Gram-positive Bacteria). Subtypes: cell wall-bounded periplasmic space [GO:0030287], outer membrane-bounded periplasmic space [GO:0030288], septal periplasm [GO:0036240] Also known as: periplasm